acetylcholine receptor binding [GO:0033130] (molecular function) Relationships: is a type of signaling receptor binding [GO:0005102] Definition: Binding to an acetylcholine receptor. Sources: GOC:mah